insulin-like growth factor receptor signaling pathway [GO:0048009] (biological process) Definition: The series of molecular signals initiated by a ligand binding to an insulin-like growth factor receptor on the surface of a target cell, and ending with the regulation of a downstream cellular process, e.g. transcription. Regulation: regulated by GO:0043567; positively regulated by positive regulation of insulin-like growth factor receptor signaling pathway [GO:0043568]; negatively regulated by GO:0043569 Sources: GOC:ceb Relationships: is a type of GO:0007169 Also known as: IGF receptor signaling pathway, IGF receptor signalling pathway